mucilage extrusion from seed coat [GO:0080001] (biological process) References: PMID:18266922 Relationships: is a type of multicellular organismal reproductive process [GO:0048609]; is part of seed germination [GO:0009845]; is part of seed development [GO:0048316] Definition: The process in which seed mucilage expands through hydration and breaks the outer cell wall that encapsulates the whole seed upon imbibition. Mucilage, mainly composed of pectins, is formed during seed development and deposited into the apoplast underneath the outer wall of the seed coat. Also known as: mucilage release from seed coat, secretion of mucilage from seed coat